{
  "term_label": "Unknown biological process",
  "gene_symbol": "ETDC",
  "gene_name": "Embryonic testis differentiation protein homolog C",
  "gene": "UniProtKB:A0A1B0GVM5",
  "term_id": "UNKNOWN:0002"
}